{
  "term_id": "GO:0006182",
  "gene_symbol": "NPR1",
  "gene_name": "Atrial natriuretic peptide receptor 1",
  "gene": "UniProtKB:P16066",
  "term_label": "cGMP biosynthetic process"
}